{
  "gene_symbol": "WIPI2",
  "term_label": "cytosol",
  "term_id": "GO:0005829",
  "gene_name": "WD repeat domain phosphoinositide-interacting protein 2",
  "gene": "UniProtKB:Q9Y4P8"
}